{
  "term_label": "regulation of postsynaptic membrane neurotransmitter receptor levels",
  "gene": "UniProtKB:Q92796",
  "gene_symbol": "DLG3",
  "gene_name": "Disks large homolog 3",
  "term_id": "GO:0099072"
}